{
  "term_label": "Golgi membrane",
  "term_id": "GO:0000139",
  "gene_name": "Guanine nucleotide exchange factor subunit RIC1",
  "gene_symbol": "RIC1",
  "gene": "UniProtKB:Q4ADV7"
}